{
  "term_label": "cytoplasm",
  "gene_symbol": "ACTBL2",
  "gene": "UniProtKB:Q562R1",
  "term_id": "GO:0005737",
  "gene_name": "Beta-actin-like protein 2"
}